regulation of interleukin-17A production [GO:0150151] (biological process) References: PMID:27901018 Sources: GOC:aruk Subtypes: negative regulation of interleukin-17A production [GO:0150152], positive regulation of interleukin-17A production [GO:0150153] Relationships: is a type of regulation of interleukin-17 production [GO:0032660]; regulates interleukin-17A production [GO:0097087] Also known as: regulation of interleukin-17A biosynthetic process Definition: Any process that modulates the frequency, rate or extent of interleukin-17A production.